DNA topoisomerase type II (double strand cut, ATP-hydrolyzing) complex [GO:0009330] (cellular component) Relationships: is a type of catalytic complex [GO:1902494] Subtypes: DNA topoisomerase IV complex [GO:0009340], DNA gyrase complex [GO:0120217] Definition: Complex that possesses DNA topoisomerase II (double strand cut, ATP-hydrolyzing) activity. Sources: GOC:bhm, GOC:krc, GOC:mah, WikiPedia:Type_II_topoisomerase